positive regulation of mucus secretion [GO:0070257] (biological process) Definition: Any process that activates or increases the frequency, rate or extent of the regulated release of mucus from a cell or a tissue. Sources: GOC:add Relationships: is a type of positive regulation of secretion [GO:0051047]; is a type of GO:0051240; is a type of regulation of mucus secretion [GO:0070255]; positively regulates mucus secretion [GO:0070254] Also known as: positive regulation of mucus production